{
  "gene": "UniProtKB:P16104",
  "term_label": "nucleosome",
  "gene_name": "Histone H2AX",
  "term_id": "GO:0000786",
  "gene_symbol": "H2AX"
}